1,2-alpha-L-fucosidase activity [GO:0047513] (molecular function) Definition: Catalysis of the reaction: H2O + methyl-2-alpha-L-fucopyranosyl-beta-D-galactoside = L-fucose + methyl beta-D-galactoside. Relationships: is a type of alpha-L-fucosidase activity [GO:0004560] Also known as: almond emulsin fucosidase II activity, 2-alpha-L-fucopyranosyl-beta-D-galactoside fucohydrolase activity, almond emulsin fucosidase activity, alpha-(1->2)-L-fucosidase activity Sources: EC:3.2.1.63, MetaCyc:12-ALPHA-L-FUCOSIDASE-RXN